{
  "gene_name": "1-phosphatidylinositol 4,5-bisphosphate phosphodiesterase beta-1",
  "term_id": "GO:0051209",
  "gene_symbol": "PLCB1",
  "gene": "UniProtKB:Q9NQ66",
  "term_label": "release of sequestered calcium ion into cytosol"
}